{
  "term_id": "GO:0097228",
  "term_label": "sperm principal piece",
  "gene_symbol": "FSCB",
  "gene_name": "Fibrous sheath CABYR-binding protein",
  "gene": "UniProtKB:Q5H9T9"
}